{
  "gene_name": "Cadherin EGF LAG seven-pass G-type receptor 1",
  "gene": "UniProtKB:Q9NYQ6",
  "term_label": "axonogenesis",
  "gene_symbol": "CELSR1",
  "term_id": "GO:0007409"
}